coniferyl aldehyde 5-hydroxylase activity [GO:0102126] (molecular function) Definition: Catalysis of the reaction: H+ + coniferyl aldehyde + NADPH + O2 = 5-hydroxy-coniferaldehyde + NADP + H2O. Sources: GOC:pz Relationships: is a type of GO:0016709